{
  "gene_name": "Heat shock 70 kDa protein 4L",
  "gene_symbol": "HSPA4L",
  "term_id": "GO:0005634",
  "gene": "UniProtKB:O95757",
  "term_label": "nucleus"
}